{
  "gene": "UniProtKB:Q5T6F0",
  "gene_name": "DDB1- and CUL4-associated factor 12",
  "term_label": "Unknown biological process",
  "term_id": "UNKNOWN:0002",
  "gene_symbol": "DCAF12"
}